{
  "gene_symbol": "CCDC60",
  "gene": "UniProtKB:Q8IWA6",
  "term_id": "UNKNOWN:0003",
  "gene_name": "Coiled-coil domain-containing protein 60",
  "term_label": "Unknown cellular component"
}